{
  "term_id": "GO:0031507",
  "gene_symbol": "MACROH2A2",
  "gene_name": "Core histone macro-H2A.2",
  "term_label": "heterochromatin formation",
  "gene": "UniProtKB:Q9P0M6"
}